{
  "term_label": "RNA nuclease activity",
  "gene_name": "Ribonuclease 8",
  "gene_symbol": "RNASE8",
  "gene": "UniProtKB:Q8TDE3",
  "term_id": "GO:0004540"
}